chloride:bicarbonate antiporter activity [GO:0140900] (molecular function) Also known as: bicarbonate:chloride antiporter activity, chloride:hydrogencarbonate antiporter activity References: PMID:10428871, PMID:16606687 Sources: RHEA:72203 Definition: Enables the transfer of a solute or solutes from one side of a membrane to the other according to the reaction: chloride(in) + HCO3-(out) = chloride(out) + HCO3-(in). Relationships: is a type of solute:inorganic anion antiporter activity [GO:0005452]; is a type of chloride transmembrane transporter activity [GO:0015108]; is a type of bicarbonate:monoatomic anion antiporter activity [GO:0140829] Subtypes: sodium,bicarbonate:chloride antiporter activity [GO:0140892]